regulation of peptidyl-L-cysteine S-palmitoylation [GO:1902662] (biological process) Relationships: is a type of regulation of protein lipidation [GO:1903059]; regulates GO:0018230 References: PMID:23444136 Sources: GOC:TermGenie, GO_REF:0000058 Subtypes: negative regulation of peptidyl-L-cysteine S-palmitoylation [GO:1902663], positive regulation of peptidyl-L-cysteine S-palmitoylation [GO:1902664] Definition: Any process that modulates the frequency, rate or extent of peptidyl-L-cysteine S-palmitoylation. Also known as: regulation of peptidyl-S-palmitoyl-L-cysteine anabolism from peptidyl-cysteine, regulation of peptidyl-S-palmitoyl-L-cysteine biosynthetic process from peptidyl-cysteine, regulation of peptidyl-S-palmitoyl-L-cysteine formation from peptidyl-cysteine, regulation of peptidyl-S-palmitoyl-L-cysteine synthesis from peptidyl-cysteine, regulation of peptidyl-cysteine S-palmitoylation